positive regulation of leukocyte cell-cell adhesion [GO:1903039] (biological process) References: PMID:21106532 Sources: GOC:BHF, GOC:TermGenie, GOC:rl, GO_REF:0000058 Also known as: positive regulation of leukocyte adhesion, positive regulation of leukocyte cell adhesion, up regulation of leukocyte adhesion, up regulation of leukocyte cell adhesion, up regulation of leukocyte cell-cell adhesion, up-regulation of leukocyte adhesion, up-regulation of leukocyte cell adhesion, up-regulation of leukocyte cell-cell adhesion, upregulation of leukocyte adhesion, upregulation of leukocyte cell adhesion, upregulation of leukocyte cell-cell adhesion, activation of leukocyte adhesion, activation of leukocyte cell adhesion, activation of leukocyte cell-cell adhesion Relationships: is a type of positive regulation of cell-cell adhesion [GO:0022409]; is a type of regulation of leukocyte cell-cell adhesion [GO:1903037]; positively regulates GO:0007159 Note: Exogenous expression of ASS1 or NOS3 in HUVECs enhances NO production and inhibits monocyte adhesion Definition: Any process that activates or increases the frequency, rate or extent of leukocyte cell-cell adhesion. Subtypes: positive regulation of T cell activation [GO:0050870], positive regulation of monocyte aggregation [GO:1900625], GO:1904996, positive regulation of thymocyte aggregation [GO:2000400], positive regulation of neutrophil aggregation [GO:2000430]